{
  "gene": "UniProtKB:Q6PID8",
  "gene_name": "Kelch domain-containing protein 10",
  "term_label": "Unknown cellular component",
  "term_id": "UNKNOWN:0003",
  "gene_symbol": "KLHDC10"
}